adenylate cyclase-inhibiting dopamine receptor signaling pathway [GO:0007195] (biological process) Regulation: regulated by regulation of adenylate cyclase-inhibiting dopamine receptor signaling pathway [GO:1904990]; negatively regulated by negative regulation of adenylate cyclase-inhibiting dopamine receptor signaling pathway [GO:1904991]; positively regulated by positive regulation of adenylate cyclase-inhibiting dopamine receptor signaling pathway [GO:1904992] Sources: GOC:dph, GOC:mah, GOC:signaling, GOC:tb Definition: An adenylate cyclase-inhibiting G protein-coupled receptor signaling pathway initiated by dopamine binding to its receptor, and ending with the regulation of a downstream cellular process. Also known as: dopamine receptor, adenylate cyclase inhibiting pathway, dopamine receptor, adenylyl cyclase inhibiting pathway, inhibition of adenylate cyclase activity by dopamine receptor signalling pathway, inhibition of adenylate cyclase activity by dopamine receptor signaling pathway Relationships: is a type of adenylate cyclase-inhibiting G protein-coupled receptor signaling pathway [GO:0007193]; is a type of G protein-coupled dopamine receptor signaling pathway [GO:0007212]